{
  "gene": "UniProtKB:Q96AQ8",
  "term_id": "GO:0030674",
  "gene_name": "Mitochondrial calcium uniporter regulator 1",
  "gene_symbol": "MCUR1",
  "term_label": "protein-macromolecule adaptor activity"
}